{
  "term_id": "GO:0008126",
  "gene": "UniProtKB:Q8WU67",
  "gene_symbol": "ABHD3",
  "gene_name": "Phospholipase ABHD3",
  "term_label": "acetylesterase activity"
}